plastid promoter transcription regulatory region sequence-specific DNA binding [GO:0001019] (molecular function) Definition: Binding to a DNA region that controls transcription by a plastid RNA polymerase. Binding may occur as a sequence specific interaction or as an interaction observed only once a factor has been recruited to the DNA by other factors. Note: plastid promoter regulatory region sequence-specific DNA binding Relationships: is a type of GO:0000976 Sources: GOC:txnOH, GOC:vw